tRNA (cytidine(32)-2'-O)-methyltransferase activity [GO:0106339] (molecular function) Definition: Catalysis of the reaction: cytidine(32) in tRNA + S-adenosyl-L-methionine = 2'-O-methylcytidine(32) in tRNA + S-adenosyl-L-homocysteine + H+. References: PMID:25404562 Sources: RHEA:42932 Also known as: tRNA (cytidine 32-2'-O)-methyltransferase activity Relationships: is a type of tRNA (cytidine) methyltransferase activity [GO:0016427]